monoatomic ion channel activity [GO:0005216] (molecular function) Relationships: is a type of monoatomic ion transmembrane transporter activity [GO:0015075]; is a type of channel activity [GO:0015267] Definition: Enables the facilitated diffusion of a monoatomic ion (by an energy-independent process) by passage through a transmembrane aqueous pore or channel without evidence for a carrier-mediated mechanism. May be either selective (it enables passage of a specific ion only) or non-selective (it enables passage of two or more ions of same charge but different size). Subtypes: voltage-gated monoatomic ion channel activity [GO:0005244], monoatomic anion channel activity [GO:0005253], GO:0005261, mechanosensitive monoatomic ion channel activity [GO:0008381], light-activated monoatomic ion channel activity [GO:0010461], GO:0015276, temperature-gated ion channel activity [GO:0097603] Also known as: ion channel activity Regulation: negatively regulated by ion channel inhibitor activity [GO:0008200]; regulated by ion channel regulator activity [GO:0099106] Sources: GOC:cy, GOC:mtg_transport, GOC:pr, ISBN:0815340729